{
  "gene": "UniProtKB:Q9BYR5",
  "gene_symbol": "KRTAP4-2",
  "term_label": "hair cycle",
  "term_id": "GO:0042633",
  "gene_name": "Keratin-associated protein 4-2"
}